histone H4K8ac reader activity [GO:0140055] (molecular function) Definition: A histone reader that recognizes a histone H4 acetylated at lysine 8. References: PMID:17996705 Also known as: H4K8ac modified histone binding Note: Note that the residue position corresponds to the canonical human H4 histone (UniProtKB:P02309); this residue is conserved across all eukaryotes. Note that the initiation methionine is cleaved, so the first residue is S1. Relationships: is a type of histone H4 reader activity [GO:0140008]